{
  "gene_symbol": "CSK",
  "gene_name": "Tyrosine-protein kinase CSK",
  "term_id": "GO:0060368",
  "gene": "UniProtKB:P41240",
  "term_label": "regulation of Fc receptor mediated stimulatory signaling pathway"
}